{
  "gene_name": "DNA damage-inducible transcript 3 protein",
  "gene": "UniProtKB:P35638",
  "term_label": "RNA polymerase II cis-regulatory region sequence-specific DNA binding",
  "term_id": "GO:0000978",
  "gene_symbol": "DDIT3"
}